lysophosphatidylcholine flippase activity [GO:0140348] (molecular function) Definition: Catalysis of the movement of lysophosphatidylcholine from the exoplasmic to the cytosolic leaflet of a membrane, using energy from the hydrolysis of ATP. Relationships: is a type of glycerophospholipid flippase activity [GO:0140333] Also known as: lysophosphatidylcholine flippase activity (exoplasmic to cytosolic leaflet) References: PMID:26945070